{
  "gene_symbol": "BAG1",
  "term_id": "GO:0005829",
  "gene_name": "BAG family molecular chaperone regulator 1",
  "term_label": "cytosol",
  "gene": "UniProtKB:Q99933"
}